U1 snRNA 3'-end processing [GO:0034473] (BP) Definition: Any process involved in forming the mature 3' end of a U1 snRNA molecule. Relationships: is a type of snRNA 3'-end processing [GO:0034472] Sources: GOC:mah Also known as: U1 snRNA 3' end processing